{
  "gene_symbol": "PIP4P2",
  "term_label": "phosphatidylinositol-4,5-bisphosphate 4-phosphatase activity",
  "gene_name": "Type 2 phosphatidylinositol 4,5-bisphosphate 4-phosphatase",
  "term_id": "GO:0034597",
  "gene": "UniProtKB:Q8N4L2"
}